{
  "gene": "UniProtKB:A0JP26",
  "gene_name": "POTE ankyrin domain family member B3",
  "term_label": "Unknown molecular function",
  "gene_symbol": "POTEB3",
  "term_id": "UNKNOWN:0001"
}